{
  "gene_name": "Zinc finger protein 892",
  "gene": "UniProtKB:A0A087WUV0",
  "gene_symbol": "ZNF892",
  "term_id": "GO:0000978",
  "term_label": "RNA polymerase II cis-regulatory region sequence-specific DNA binding"
}